{
  "gene_name": "Germ cell-specific gene 1 protein",
  "term_label": "Unknown biological process",
  "gene_symbol": "GSG1",
  "gene": "UniProtKB:Q2KHT4",
  "term_id": "UNKNOWN:0002"
}